{
  "term_id": "GO:0000978",
  "gene_symbol": "FOXC1",
  "term_label": "RNA polymerase II cis-regulatory region sequence-specific DNA binding",
  "gene_name": "Forkhead box protein C1",
  "gene": "UniProtKB:Q12948"
}